{
  "gene_name": "Excitatory amino acid transporter 1",
  "term_id": "GO:0098712",
  "gene": "UniProtKB:P43003",
  "gene_symbol": "SLC1A3",
  "term_label": "L-glutamate import across plasma membrane"
}